positive regulation of cellular senescence [GO:2000774] (biological process) Definition: Any process that activates or increases the frequency, rate or extent of cellular senescence. Sources: GOC:BHF Relationships: is a type of positive regulation of cellular process [GO:0048522]; is a type of regulation of cellular senescence [GO:2000772]; positively regulates cellular senescence [GO:0090398]